{
  "gene_name": "Polycomb protein SUZ12",
  "gene_symbol": "SUZ12",
  "term_label": "Unknown biological process",
  "gene": "UniProtKB:Q15022",
  "term_id": "UNKNOWN:0002"
}